endonucleolytic cleaveage between 4.5S rRNA and 5S rRNA of tetracistronic rRNA transcript (SSU-rRNA, LSU-rRNA, 4.5S-rRNA, 5S-rRNA) [GO:0002104] (biological process) Definition: Endonucleolytic cleavage between the 5S rRNA and the 4.5S rRNA of an rRNA molecule originally produced as a tetracistronic rRNA transcript that contains the Small Subunit (SSU) rRNA, Large Subunit (LSU) the 4.5S rRNA, and the 5S rRNA in that order from 5' to 3' along the primary transcript. Note that the use of the word tetracistronic refers only to the number of mature rRNA molecules which will be produced from the primary transcript and ignores tRNAs that may also be present within the primary transcript. Sources: GOC:curators Relationships: is a type of endonucleolytic cleavage of tetracistronic rRNA transcript (SSU-rRNA, LSU-rRNA, 4.5S-rRNA, 5S-rRNA) [GO:0002103]